phenylethylamine biosynthetic process [GO:0042444] (biological process) Also known as: phenylethylamine anabolism, phenylethylamine biosynthesis, phenylethylamine formation, phenylethylamine synthesis Relationships: is a type of biogenic amine biosynthetic process [GO:0042401]; is a type of phenylethylamine metabolic process [GO:0042443]; is a type of GO:1901162 Definition: The chemical reactions and pathways resulting in the formation of phenylethylamine, an amine with pharmacological properties similar to those of amphetamine, occurs naturally as a neurotransmitter in the brain, and is present in chocolate and oil of bitter almonds. Sources: GOC:jl, ISBN:0395825172